{
  "gene_symbol": "OXGR1",
  "term_label": "G protein-coupled receptor signaling pathway",
  "gene": "UniProtKB:Q96P68",
  "gene_name": "2-oxoglutarate receptor 1",
  "term_id": "GO:0007186"
}